{
  "gene": "UniProtKB:Q13214",
  "gene_symbol": "SEMA3B",
  "term_id": "GO:0030335",
  "term_label": "positive regulation of cell migration",
  "gene_name": "Semaphorin-3B"
}